{
  "gene": "UniProtKB:P62820",
  "term_label": "autophagosome assembly",
  "gene_name": "Ras-related protein Rab-1A",
  "term_id": "GO:0000045",
  "gene_symbol": "RAB1A"
}